{
  "gene": "UniProtKB:Q15057",
  "gene_symbol": "ACAP2",
  "gene_name": "Arf-GAP with coiled-coil, ANK repeat and PH domain-containing protein 2",
  "term_label": "Unknown molecular function",
  "term_id": "UNKNOWN:0001"
}